{
  "gene_symbol": "PROM1",
  "term_id": "GO:0016324",
  "term_label": "apical plasma membrane",
  "gene_name": "Prominin-1",
  "gene": "UniProtKB:O43490"
}